{
  "gene": "UniProtKB:P46098",
  "term_id": "GO:0005231",
  "gene_name": "5-hydroxytryptamine receptor 3A",
  "gene_symbol": "HTR3A",
  "term_label": "excitatory extracellular ligand-gated monoatomic ion channel activity"
}